response to alkaloid [GO:0043279] (biological process) Definition: Any process that results in a change in state or activity of a cell or an organism (in terms of movement, secretion, enzyme production, gene expression, etc.) as a result of an alkaloid stimulus. Alkaloids are a large group of nitrogenous substances found in naturally in plants, many of which have extracts that are pharmacologically active. Sources: GOC:jl Relationships: is_a response to nitrogen compound [GO:1901698] Subtypes: response to isoquinoline alkaloid [GO:0014072], response to tropane [GO:0014073], GO:0031000, response to cocaine [GO:0042220], cellular response to alkaloid [GO:0071312], response to staurosporine [GO:0072733], response to camptothecin [GO:1901563]